proteasome core complex binding [GO:1904854] (molecular function) Also known as: macropain binding, 20S core complex binding, 20S proteasome binding, PA28gamma-20S proteasome binding References: PMID:16096059 Sources: GOC:TermGenie Relationships: is a type of protein-containing complex binding [GO:0044877] Definition: Binding to a proteasome core complex.